{
  "term_id": "UNKNOWN:0003",
  "term_label": "Unknown cellular component",
  "gene_name": "Uncharacterized protein C11orf21",
  "gene": "UniProtKB:Q9P2W6",
  "gene_symbol": "C11orf21"
}